{
  "gene": "UniProtKB:P35573",
  "term_label": "Unknown cellular component",
  "term_id": "UNKNOWN:0003",
  "gene_name": "Glycogen debranching enzyme",
  "gene_symbol": "AGL"
}